{
  "term_id": "UNKNOWN:0002",
  "term_label": "Unknown biological process",
  "gene_name": "Transmembrane protein 215",
  "gene_symbol": "TMEM215",
  "gene": "UniProtKB:Q68D42"
}